{
  "gene_symbol": "APOA1",
  "gene_name": "Apolipoprotein A-I",
  "term_label": "cholesterol metabolic process",
  "gene": "UniProtKB:P02647",
  "term_id": "GO:0008203"
}